xanthophyll metabolic process [GO:0016122] (biological process) Relationships: is a type of carotenoid metabolic process [GO:0016116] Subtypes: xanthophyll cycle [GO:0010028], GO:0016123, GO:0016124 Sources: ISBN:0198547684 Also known as: xanthophyll metabolism Definition: The chemical reactions and pathways involving xanthophylls, oxygen-containing carotenoids.